negative regulation of viral process [GO:0048525] (biological process) Definition: Any process that stops, prevents, or reduces the frequency, rate or extent of a multi-organism process in which a virus is a participant. Relationships: is a type of GO:0048519; is a type of regulation of viral process [GO:0050792]; negatively regulates viral process [GO:0016032] Sources: GOC:bf, GOC:jl Subtypes: negative regulation of viral transcription [GO:0032897], negative regulation by host of viral glycoprotein metabolic process [GO:0044871], negative regulation of viral genome replication [GO:0045071], negative regulation by virus of viral protein levels in host cell [GO:0046725], GO:1903901, negative regulation of fusion of virus membrane with host plasma membrane [GO:1903914], negative regulation of viral translation [GO:1904972] Also known as: down regulation of viral life cycle, down-regulation of viral life cycle, downregulation of viral life cycle, inhibition of viral life cycle, negative regulation of viral life cycle, negative regulation of viral reproduction